cyclic threonylcarbamoyladenosine biosynthetic process [GO:0061504] (biological process) References: PMID:23242255 Definition: The chemical reactions and pathways resulting in the formation of cyclic threonylcarbamoyladenosine, a modified nucleoside found in some tRNA molecules. Relationships: is a type of tRNA modification [GO:0006400]